ESCRT complex disassembly [GO:1904896] (biological process) Relationships: is a type of GO:0032984 Also known as: endosomal sorting complex required for transport disassembly Subtypes: ESCRT III complex disassembly [GO:1904903] Definition: The disaggregation of an ESCRT complex into its constituent components. References: PMID:21118109 Sources: GOC:PARL, GOC:TermGenie, GOC:pad, GO_REF:0000079